{
  "gene_name": "High mobility group protein B4",
  "term_id": "GO:0005634",
  "term_label": "nucleus",
  "gene_symbol": "HMGB4",
  "gene": "UniProtKB:Q8WW32"
}